cell-cell adhesion involved in gastrulation [GO:0070586] (biological process) References: PMID:19091770 Sources: GOC:dsf Relationships: is a type of cell-cell adhesion [GO:0098609]; is part of GO:0007369 Subtypes: GO:0003370 Regulation: regulated by regulation of cell-cell adhesion involved in gastrulation [GO:0070587] Definition: The attachment of one cell to another cell affecting gastrulation.